{
  "term_label": "RNA polymerase II cis-regulatory region sequence-specific DNA binding",
  "gene": "UniProtKB:Q15697",
  "term_id": "GO:0000978",
  "gene_name": "Zinc finger protein 174",
  "gene_symbol": "ZNF174"
}